4-hydroxybenzoate-CoA ligase activity [GO:0018859] (molecular function) Also known as: 4-hydroxybenzoate-CoA synthetase activity, 4-hydroxybenzoate-coenzyme A ligase (AMP-forming), 4-hydroxybenzoate:CoA ligase (AMP-forming), 4-hydroxybenzoyl coenzyme A synthetase activity, 4-hydroxybenzoyl-CoA ligase activity Sources: EC:6.2.1.27 Definition: Catalysis of the reaction: ATP + 4-hydroxybenzoate + CoA = AMP + diphosphate + 4-hydroxybenzoyl-CoA. Relationships: is a type of GO:0016405; is a type of acid-thiol ligase activity [GO:0016878]